{
  "gene_symbol": "GIMAP6",
  "term_id": "UNKNOWN:0002",
  "term_label": "Unknown biological process",
  "gene_name": "GTPase IMAP family member 6",
  "gene": "UniProtKB:Q6P9H5"
}